{
  "gene": "UniProtKB:Q7Z392",
  "term_label": "Unknown molecular function",
  "gene_symbol": "TRAPPC11",
  "gene_name": "Trafficking protein particle complex subunit 11",
  "term_id": "UNKNOWN:0001"
}